retinoid metabolic process [GO:0001523] (biological process) Subtypes: GO:0006776, retinol metabolic process [GO:0042572], GO:0042573, retinal metabolic process [GO:0042574] Sources: ISBN:0198506732 Definition: The chemical reactions and pathways involving retinoids, any member of a class of isoprenoids that contain or are derived from four prenyl groups linked head-to-tail. Retinoids include retinol and retinal and structurally similar natural derivatives or synthetic compounds, but need not have vitamin A activity. Relationships: is a type of diterpenoid metabolic process [GO:0016101] Also known as: retinoid metabolism